{
  "term_label": "growth factor activity",
  "term_id": "GO:0008083",
  "gene": "UniProtKB:P26441",
  "gene_symbol": "CNTF",
  "gene_name": "Ciliary neurotrophic factor"
}